{
  "gene_name": "Olfactory receptor 5M8",
  "gene_symbol": "OR5M8",
  "gene": "UniProtKB:Q8NGP6",
  "term_id": "GO:0005549",
  "term_label": "odorant binding"
}